{
  "term_id": "UNKNOWN:0002",
  "gene_name": "Olfactory receptor 8U9",
  "term_label": "Unknown biological process",
  "gene_symbol": "OR8U9",
  "gene": "UniProtKB:P0C7N5"
}